{
  "term_label": "DNA-binding transcription factor activity, RNA polymerase II-specific",
  "gene_name": "Homeobox protein Hox-C5",
  "term_id": "GO:0000981",
  "gene_symbol": "HOXC5",
  "gene": "UniProtKB:Q00444"
}